{
  "term_id": "GO:0006414",
  "gene_name": "Eukaryotic translation initiation factor 5A-1-like",
  "term_label": "translational elongation",
  "gene_symbol": "EIF5AL1",
  "gene": "UniProtKB:Q6IS14"
}